acyl-CoA 11-(E)-desaturase activity [GO:0050600] (molecular function) Definition: Catalysis of the reaction: an 11,12-saturated fatty acyl-CoA + 2 Fe(II)-[cytochrome b5] + 2 H+ + O2 = an (11E)-delta11-fatty acyl-CoA + 2 Fe(III)-[cytochrome b5] + 2 H2O. Sources: RHEA:46396 Also known as: acyl-CoA delta11-desaturase activity, myristoyl-CoA 11-(E) desaturase activity Relationships: is a type of acyl-CoA desaturase activity [GO:0016215]